{
  "term_label": "Unknown molecular function",
  "gene": "UniProtKB:Q9P2G3",
  "gene_name": "Kelch-like protein 14",
  "term_id": "UNKNOWN:0001",
  "gene_symbol": "KLHL14"
}